protopine 6-monooxygenase activity [GO:0047087] (molecular function) Sources: RHEA:22644 Also known as: protopine 6-hydroxylase activity, protopine,NADPH:oxygen oxidoreductase (6-hydroxylating) Relationships: is a type of GO:0016709 Definition: Catalysis of the reaction: O2 + protopine + reduced [NADPH--hemoprotein reductase] = 6-hydroxyprotopine + H+ + H2O + oxidized [NADPH--hemoprotein reductase].